{
  "gene_symbol": "MIXL1",
  "gene_name": "Homeobox protein MIXL1",
  "gene": "UniProtKB:Q9H2W2",
  "term_label": "Unknown cellular component",
  "term_id": "UNKNOWN:0003"
}